{
  "term_label": "Unknown cellular component",
  "gene": "UniProtKB:Q5T7N8",
  "term_id": "UNKNOWN:0003",
  "gene_name": "Protein FAM27D1",
  "gene_symbol": "FAM27D1"
}